{
  "term_id": "UNKNOWN:0001",
  "gene_symbol": "APOBEC4",
  "term_label": "Unknown molecular function",
  "gene_name": "Putative C-U-editing enzyme APOBEC-4",
  "gene": "UniProtKB:Q8WW27"
}